{
  "gene_symbol": "SBK3",
  "term_id": "UNKNOWN:0002",
  "term_label": "Unknown biological process",
  "gene_name": "Uncharacterized serine_threonine-protein kinase SBK3",
  "gene": "UniProtKB:P0C264"
}